{
  "gene_name": "Zinc finger protein 705A",
  "term_id": "GO:0000981",
  "gene_symbol": "ZNF705A",
  "gene": "UniProtKB:Q6ZN79",
  "term_label": "DNA-binding transcription factor activity, RNA polymerase II-specific"
}